{
  "gene": "UniProtKB:Q9NRW1",
  "term_label": "GTPase activity",
  "gene_name": "Ras-related protein Rab-6B",
  "term_id": "GO:0003924",
  "gene_symbol": "RAB6B"
}